Kv4.3-KChIP1 channel complex [GO:0071196] (cellular component) Definition: A voltage-gated potassium channel complex that contains the Kv channel interacting protein KChIP1 associated with the channel via interaction with the Kv alpha subunit 4.3. References: PMID:15356203 Relationships: is a type of GO:0008076